alpha-1,4-N-acetylgalactosaminyltransferase activity [GO:0035248] (molecular function) Relationships: is a type of GO:0008376 References: PMID:15130086 Also known as: alpha-1,4-GalNAc transferase activity Definition: Catalysis of the transfer of an N-acetylgalactosaminyl residue from UDP-N-acetyl-galactosamine to an acceptor molecule, forming an alpha-1,4 linkage.